{
  "gene_name": "Gamma-aminobutyric acid receptor-associated protein",
  "gene_symbol": "GABARAP",
  "term_label": "ubiquitin protein ligase binding",
  "term_id": "GO:0031625",
  "gene": "UniProtKB:O95166"
}